{
  "gene_symbol": "PPP2CA",
  "gene_name": "Serine_threonine-protein phosphatase 2A catalytic subunit alpha isoform",
  "term_label": "protein serine/threonine phosphatase activity",
  "gene": "UniProtKB:P67775",
  "term_id": "GO:0004722"
}